{
  "gene_symbol": "ZNF510",
  "gene_name": "Zinc finger protein 510",
  "term_label": "regulation of transcription by RNA polymerase II",
  "gene": "UniProtKB:Q9Y2H8",
  "term_id": "GO:0006357"
}